phytochromobilin:ferredoxin oxidoreductase activity [GO:0050619] (molecular function) Also known as: (3Z)-phytochromobilin:ferredoxin oxidoreductase activity, HY2, P-Phi-B synthase activity, PFB synthase activity, PPhiB synthase activity, phytochromobilin synthase activity Relationships: is a type of oxidoreductase activity, acting on the CH-CH group of donors, iron-sulfur protein as acceptor [GO:0016636] Sources: EC:1.3.7.4, MetaCyc:1.3.7.4-RXN Definition: Catalysis of the reaction: (3Z)-phytochromobilin + oxidized ferredoxin = biliverdin IXa + reduced ferredoxin.